positive regulation of kinetochore assembly [GO:1905561] (BP) Relationships: is a type of positive regulation of protein-containing complex assembly [GO:0031334]; is a type of regulation of kinetochore assembly [GO:0090234]; is a type of positive regulation of organelle assembly [GO:1902117]; is a type of positive regulation of chromosome organization [GO:2001252]; positively regulates kinetochore assembly [GO:0051382] References: PMID:18765790 Sources: GOC:TermGenie, GO_REF:0000058 Also known as: up regulation of kinetochore assembly, up-regulation of kinetochore assembly, upregulation of kinetochore assembly, activation of centromere and kinetochore complex maturation, activation of centromere/kinetochore complex maturation, activation of chromosome-kinetochore attachment, activation of kinetochore assembly, positive regulation of NMS complex assembly, positive regulation of centromere and kinetochore complex maturation, positive regulation of centromere/kinetochore complex maturation, positive regulation of chromosome-kinetochore attachment, up regulation of centromere and kinetochore complex maturation, up regulation of centromere/kinetochore complex maturation, up regulation of chromosome-kinetochore attachment, up-regulation of centromere and kinetochore complex maturation, up-regulation of centromere/kinetochore complex maturation, up-regulation of chromosome-kinetochore attachment, upregulation of centromere and kinetochore complex maturation, upregulation of centromere/kinetochore complex maturation, upregulation of chromosome-kinetochore attachment, activation of kinetochore formation, positive regulation of kinetochore formation, up regulation of kinetochore formation, up-regulation of kinetochore formation, upregulation of kinetochore formation Definition: Any process that activates or increases the frequency, rate or extent of kinetochore assembly.